{
  "term_id": "GO:0061799",
  "gene_name": "Molybdenum cofactor biosynthesis protein 1",
  "gene_symbol": "MOCS1",
  "term_label": "cyclic pyranopterin monophosphate synthase activity",
  "gene": "UniProtKB:Q9NZB8"
}